{
  "gene_name": "Insulin receptor",
  "term_id": "GO:0005899",
  "gene_symbol": "INSR",
  "gene": "UniProtKB:P06213",
  "term_label": "insulin receptor complex"
}